{
  "term_id": "GO:0005886",
  "gene_name": "Amiloride-sensitive sodium channel subunit gamma",
  "gene": "UniProtKB:P51170",
  "term_label": "plasma membrane",
  "gene_symbol": "SCNN1G"
}